VEGF-activated platelet-derived growth factor receptor-beta signaling pathway [GO:0038088] (BP) References: PMID:17470632 Sources: GOC:signaling Relationships: is a type of platelet-derived growth factor receptor-beta signaling pathway [GO:0035791]; is a type of VEGF-activated platelet-derived growth factor receptor signaling pathway [GO:0038086] Definition: The series of molecular signals initiated by vascular endothelial growth factor (VEGF) binding to a beta-type platelet-derived growth factor receptor (PDGFR) on the surface of a cell, and ending with the regulation of a downstream cellular process, e.g. transcription. Also known as: VEGF-activated PDGFRbeta signalling pathway, VEGF-activated platelet-derived growth factor receptor-beta signalling pathway, VEGF/PDGFRbeta signaling pathway, vascular endothelial growth factor-activated platelet-derived growth factor receptor-beta signaling pathway, VEGF-A/PDGFRbeta signaling